{
  "gene_name": "Colipase-like protein 2",
  "term_id": "UNKNOWN:0003",
  "gene_symbol": "CLPSL2",
  "term_label": "Unknown cellular component",
  "gene": "UniProtKB:Q6UWE3"
}